{
  "term_label": "olfactory receptor activity",
  "gene_name": "Olfactory receptor 52N1",
  "term_id": "GO:0004984",
  "gene_symbol": "OR52N1",
  "gene": "UniProtKB:Q8NH53"
}